{
  "term_id": "GO:0000977",
  "gene_name": "Double homeobox protein 4-like protein 6",
  "term_label": "RNA polymerase II transcription regulatory region sequence-specific DNA binding",
  "gene": "UniProtKB:P0CJ89",
  "gene_symbol": "DUX4L6"
}